{
  "term_id": "GO:0005246",
  "gene": "UniProtKB:Q9P246",
  "gene_name": "Stromal interaction molecule 2",
  "term_label": "calcium channel regulator activity",
  "gene_symbol": "STIM2"
}